atrial septum development [GO:0003283] (biological process) Definition: The progression of the atrial septum over time, from its initial formation to the mature structure. Sources: GOC:mtg_heart Relationships: is a type of cardiac septum development [GO:0003279]; is part of GO:0003230 Subtypes: septum primum development [GO:0003284], septum secundum development [GO:0003285], atrial septum intermedium development [GO:0003286]